{
  "term_id": "GO:0008009",
  "gene_name": "C-C motif chemokine 23",
  "term_label": "chemokine activity",
  "gene_symbol": "CCL23",
  "gene": "UniProtKB:P55773"
}